{
  "term_label": "endocytic recycling",
  "gene_name": "Sorting nexin-3",
  "gene": "UniProtKB:O60493",
  "gene_symbol": "SNX3",
  "term_id": "GO:0032456"
}